{
  "term_id": "UNKNOWN:0001",
  "gene_symbol": "AIPL1",
  "gene_name": "Aryl-hydrocarbon-interacting protein-like 1",
  "gene": "UniProtKB:Q9NZN9",
  "term_label": "Unknown molecular function"
}